G protein-coupled acetylcholine receptor signaling pathway involved in heart process [GO:0086093] (biological process) Also known as: G-protein coupled acetylcholine receptor signaling pathway involved in heart process, G-protein coupled acetylcholine receptor signalling pathway involved in heart process, M2 receptor signaling pathway involved in heart process, muscarinic receptor signaling pathway involved in heart process Subtypes: G protein-coupled acetylcholine receptor signaling pathway involved in negative regulation of heart rate [GO:0086033] Definition: A G protein-coupled acetylcholine receptor signaling pathway, which contributes to a circulatory system process carried out by the heart. Sources: GOC:BHF, GOC:mtg_cardiac_conduct_nov11 Relationships: is a type of G protein-coupled acetylcholine receptor signaling pathway [GO:0007213]; is a type of G protein-coupled receptor signaling pathway involved in heart process [GO:0086103]